{
  "term_label": "cytoplasm",
  "gene": "UniProtKB:O43353",
  "term_id": "GO:0005737",
  "gene_name": "Receptor-interacting serine_threonine-protein kinase 2",
  "gene_symbol": "RIPK2"
}